{
  "gene": "UniProtKB:Q8IX94",
  "term_label": "Unknown molecular function",
  "gene_symbol": "CTAGE4",
  "gene_name": "cTAGE family member 4",
  "term_id": "UNKNOWN:0001"
}